{
  "term_id": "GO:1901981",
  "gene_name": "Pleckstrin homology domain-containing family N member 1",
  "gene_symbol": "PLEKHN1",
  "gene": "UniProtKB:Q494U1",
  "term_label": "phosphatidylinositol phosphate binding"
}